male courtship behavior, veined wing extension [GO:0048065] (BP) Relationships: is a type of male courtship behavior [GO:0008049] Subtypes: male courtship behavior, veined wing vibration [GO:0016545] Sources: GOC:jid, GOC:mtg_sensu Also known as: male courtship behavior, wing extension, male courtship behaviour, wing extension, male courtship behaviour, veined wing extension Definition: The process during courtship where the male insect extends his wings. An example of this process is found in Drosophila melanogaster.